{
  "term_label": "Unknown cellular component",
  "term_id": "UNKNOWN:0003",
  "gene_symbol": "ZFTA",
  "gene": "UniProtKB:C9JLR9",
  "gene_name": "Zinc finger translocation-associated protein"
}